{
  "term_label": "extracellular matrix organization",
  "gene": "UniProtKB:Q8WXS8",
  "gene_symbol": "ADAMTS14",
  "term_id": "GO:0030198",
  "gene_name": "A disintegrin and metalloproteinase with thrombospondin motifs 14"
}